{
  "gene": "UniProtKB:Q86WA8",
  "gene_symbol": "LONP2",
  "term_label": "protein processing",
  "term_id": "GO:0016485",
  "gene_name": "Lon protease homolog 2, peroxisomal"
}